{
  "gene_name": "Membrane-associated guanylate kinase, WW and PDZ domain-containing protein 3",
  "gene_symbol": "MAGI3",
  "term_id": "GO:0005911",
  "term_label": "cell-cell junction",
  "gene": "UniProtKB:Q5TCQ9"
}